{
  "term_id": "GO:0016907",
  "gene_name": "Muscarinic acetylcholine receptor M5",
  "term_label": "G protein-coupled acetylcholine receptor activity",
  "gene": "UniProtKB:P08912",
  "gene_symbol": "CHRM5"
}